{
  "gene": "UniProtKB:Q04206",
  "term_label": "positive regulation of transcription by RNA polymerase II",
  "gene_symbol": "RELA",
  "term_id": "GO:0045944",
  "gene_name": "Transcription factor p65"
}